{
  "term_id": "GO:0004144",
  "gene": "UniProtKB:Q86VF5",
  "gene_symbol": "MOGAT3",
  "gene_name": "2-acylglycerol O-acyltransferase 3",
  "term_label": "diacylglycerol O-acyltransferase activity"
}